{
  "gene_name": "F-box_WD repeat-containing protein 10",
  "term_id": "UNKNOWN:0002",
  "gene_symbol": "FBXW10",
  "gene": "UniProtKB:Q5XX13",
  "term_label": "Unknown biological process"
}